{
  "gene": "UniProtKB:B7U540",
  "term_id": "GO:0005886",
  "gene_symbol": "KCNJ18",
  "term_label": "plasma membrane",
  "gene_name": "Inward rectifier potassium channel 18"
}